{
  "term_label": "regulation of gene expression",
  "term_id": "GO:0010468",
  "gene": "UniProtKB:A6NI03",
  "gene_symbol": "TRIM64B",
  "gene_name": "Putative tripartite motif-containing protein 64B"
}